{
  "gene_symbol": "ARMCX5",
  "gene_name": "Armadillo repeat-containing X-linked protein 5",
  "gene": "UniProtKB:Q6P1M9",
  "term_id": "UNKNOWN:0003",
  "term_label": "Unknown cellular component"
}